positive regulation of developmental growth [GO:0048639] (biological process) Subtypes: positive regulation of multicellular organism growth [GO:0040018], positive regulation of skeletal muscle tissue regeneration [GO:0043415], positive regulation of imaginal disc growth [GO:0045572], GO:0045773, positive regulation of synaptic assembly at neuromuscular junction [GO:0045887], positive regulation of organ growth [GO:0046622], GO:0048633, GO:0048672, GO:0048687, positive regulation of unidimensional cell growth [GO:0051512], GO:0060504, positive regulation of convergent extension involved in axis elongation [GO:1901234], positive regulation of root hair elongation [GO:1902892], positive regulation of chondrocyte hypertrophy [GO:1903043], positive regulation of dendrite extension [GO:1903861], positive regulation of epithelium regeneration [GO:1905043], GO:1905180, positive regulation of developmental vegetative growth [GO:1905615], positive regulation of antral ovarian follicle growth [GO:2000388] Definition: Any process that activates, maintains or increases the rate of developmental growth. Sources: GOC:go_curators Relationships: is_a GO:0045927; is_a regulation of developmental growth [GO:0048638]; is a type of GO:0051094; RO_0002213 GO:0048589 Also known as: up regulation of developmental growth, up-regulation of developmental growth, upregulation of developmental growth, activation of developmental growth, stimulation of developmental growth